{
  "gene": "UniProtKB:Q9NZC9",
  "term_label": "nuclear replication fork",
  "gene_name": "SWI_SNF-related matrix-associated actin-dependent regulator of chromatin subfamily A-like protein 1",
  "term_id": "GO:0043596",
  "gene_symbol": "SMARCAL1"
}